{
  "term_id": "GO:0003924",
  "gene_name": "Guanylate-binding protein 5",
  "gene_symbol": "GBP5",
  "gene": "UniProtKB:Q96PP8",
  "term_label": "GTPase activity"
}